{
  "gene_name": "Stonin-2",
  "gene_symbol": "STON2",
  "term_label": "regulation of endocytosis",
  "term_id": "GO:0030100",
  "gene": "UniProtKB:Q8WXE9"
}